post-transcriptional gene silencing [GO:0016441] (biological process) Regulation: RO_0002211 by regulation of post-transcriptional gene silencing [GO:0060147]; positively regulated by positive regulation of post-transcriptional gene silencing [GO:0060148]; negatively regulated by negative regulation of post-transcriptional gene silencing [GO:0060149] Definition: The inactivation of gene expression that occurs after transcription. Subtypes: GO:0035194, global gene silencing by mRNA cleavage [GO:0098795], target-directed miRNA degradation [GO:0140958] Relationships: is a type of post-transcriptional regulation of gene expression [GO:0010608]; is a type of negative regulation of gene expression [GO:0010629] Also known as: PTGS, posttranscriptional gene silencing References: PMID:15020054 Sources: GOC:mah